{
  "term_id": "UNKNOWN:0002",
  "term_label": "Unknown biological process",
  "gene_symbol": "IRAG1",
  "gene": "UniProtKB:Q9Y6F6",
  "gene_name": "Inositol 1,4,5-triphosphate receptor associated 1"
}